EP2 subtype prostaglandin E2 receptor binding [GO:0031865] (molecular function) Also known as: prostanoid EP2 receptor binding, EP2 subtype prostaglandin E2 receptor ligand Definition: Binding to an EP2 subtype prostaglandin E2 receptor. Relationships: is a type of prostanoid receptor binding [GO:0031862] Sources: GOC:mah, GOC:nln